{
  "term_id": "GO:0006874",
  "term_label": "intracellular calcium ion homeostasis",
  "gene_name": "Sodium_potassium_calcium exchanger 3",
  "gene": "UniProtKB:Q9HC58",
  "gene_symbol": "SLC24A3"
}